negative regulation of horizontal cell localization [GO:1902873] (biological process) Definition: Any process that stops, prevents or reduces the frequency, rate or extent of horizontal cell localization. Also known as: down regulation of horizontal cell localisation, down regulation of horizontal cell localization, down regulation of horizontal cell positioning, down regulation of laminar positioning of retinal horizontal cell, down regulation of retinal horizontal cell positioning, down-regulation of horizontal cell localisation, down-regulation of horizontal cell localization, down-regulation of horizontal cell positioning, down-regulation of laminar positioning of retinal horizontal cell, down-regulation of retinal horizontal cell positioning, downregulation of horizontal cell localisation, downregulation of horizontal cell localization, downregulation of horizontal cell positioning, downregulation of laminar positioning of retinal horizontal cell, downregulation of retinal horizontal cell positioning, negative regulation of horizontal cell localisation, negative regulation of horizontal cell positioning, negative regulation of laminar positioning of retinal horizontal cell, negative regulation of retinal horizontal cell positioning, inhibition of horizontal cell localisation, inhibition of horizontal cell localization, inhibition of horizontal cell positioning, inhibition of laminar positioning of retinal horizontal cell, inhibition of retinal horizontal cell positioning References: PMID:16872597 Sources: GOC:TermGenie, GOC:mr, GO_REF:0000058 Relationships: is a type of negative regulation of cellular process [GO:0048523]; is a type of regulation of horizontal cell localization [GO:1902872]; negatively regulates horizontal cell localization [GO:0035852]